{
  "gene_symbol": "TUBB1",
  "term_label": "GTP binding",
  "gene": "UniProtKB:Q9H4B7",
  "gene_name": "Tubulin beta-1 chain",
  "term_id": "GO:0005525"
}